{
  "term_id": "GO:0006850",
  "gene": "UniProtKB:Q9Y5U8",
  "term_label": "pyruvate import into mitochondria",
  "gene_symbol": "MPC1",
  "gene_name": "Mitochondrial pyruvate carrier 1"
}